{
  "gene_name": "HAUS augmin-like complex subunit 2",
  "term_label": "Unknown molecular function",
  "gene_symbol": "HAUS2",
  "gene": "UniProtKB:Q9NVX0",
  "term_id": "UNKNOWN:0001"
}